hemoglobin alpha binding [GO:0031721] (MF) Definition: Binding to a hemoglobin alpha chain. Sources: GOC:mah Relationships: is a type of hemoglobin binding [GO:0030492]